{
  "gene": "UniProtKB:Q8NEZ5",
  "gene_symbol": "FBXO22",
  "term_id": "UNKNOWN:0003",
  "gene_name": "F-box only protein 22",
  "term_label": "Unknown cellular component"
}